{
  "term_label": "cytoplasm",
  "gene_symbol": "AGO2",
  "term_id": "GO:0005737",
  "gene_name": "Protein argonaute-2",
  "gene": "UniProtKB:Q9UKV8"
}